{
  "gene_symbol": "LCE3C",
  "gene_name": "Late cornified envelope protein 3C",
  "term_id": "UNKNOWN:0002",
  "term_label": "Unknown biological process",
  "gene": "UniProtKB:Q5T5A8"
}